{
  "term_label": "Unknown biological process",
  "gene_symbol": "LGALS14",
  "term_id": "UNKNOWN:0002",
  "gene": "UniProtKB:Q8TCE9",
  "gene_name": "Placental protein 13-like"
}